acyl-CoA 15-desaturase activity [GO:0102988] (molecular function) Definition: Catalysis of the reaction: (9Z,12Z)-hexadecadienoyl-CoA + O2 + a reduced electron acceptor = 9,12,15-cis-hexadecatrienoyl-CoA + 2 H2O + an oxidized electron acceptor. Also known as: 9,12-cis-hexadecadienoic acid delta 15 desaturase activity Relationships: is a type of acyl-CoA desaturase activity [GO:0016215] Sources: EC:1.14.19.13